modulation of formation of structure involved in a symbiotic process [GO:0044145] (biological process) Sources: GOC:jl, GOC:pamgo_curators Note: This term partially replaces the obsolete term 'modulation of growth or development of symbiont during interaction with host ; GO:0075338'. See also 'modulation of growth of symbiont during interaction with host ; GO:0044144'. Subtypes: GO:0044127, negative regulation of formation of structure involved in a symbiotic process [GO:0044147], positive regulation of formation of structure involved in a symbiotic process [GO:0044149], regulation of formation by symbiont of haustorium for nutrient acquisition from host [GO:0075045], modulation of symbiont haustorium neck formation for entry into host [GO:0075198], regulation of penetration hypha formation [GO:0075202], GO:0075329 Definition: Any process that modulates the frequency, rate or extent of the progression of an organism from an initial condition to a later condition, occurring in, on or near the exterior of its host organism. Relationships: is_a GO:0050789; RO_0002211 formation of structure involved in a symbiotic process [GO:0044111] Also known as: modulation of development of symbiont during interaction with host, modulation of development of symbiont involved in interaction with host